fear-induced aggressive behavior [GO:0002122] (biological process) Definition: Aggressive behavior associated with attempts to flee from a threat. Relationships: is_a aggressive behavior [GO:0002118] Sources: GOC:hjd Also known as: fear-induced aggression